{
  "gene": "UniProtKB:P30559",
  "term_label": "maternal process involved in parturition",
  "gene_symbol": "OXTR",
  "gene_name": "Oxytocin receptor",
  "term_id": "GO:0060137"
}